deoxynucleoside triphosphate hydrolase activity [GO:0106375] (molecular function) Definition: Catalysis of the reaction: dNTP + H2O = 2'-deoxynucleoside + H+ + triphosphate. Relationships: is_a triphosphoric monoester hydrolase activity [GO:0016793] Sources: RHEA:46148